{
  "term_label": "protein serine/threonine kinase activity",
  "gene": "UniProtKB:Q13043",
  "term_id": "GO:0004674",
  "gene_symbol": "STK4",
  "gene_name": "Serine_threonine-protein kinase 4"
}